{
  "gene_name": "Sodium_hydrogen exchanger 6",
  "gene_symbol": "SLC9A6",
  "term_id": "GO:0071805",
  "term_label": "potassium ion transmembrane transport",
  "gene": "UniProtKB:Q92581"
}